{
  "gene_name": "Potassium voltage-gated channel subfamily H member 6",
  "gene_symbol": "KCNH6",
  "gene": "UniProtKB:Q9H252",
  "term_label": "potassium ion transmembrane transport",
  "term_id": "GO:0071805"
}